glutamate secretion, neurotransmission [GO:0061535] (biological process) Definition: The controlled release of glutamate by a cell, in which the glutamate acts as a neurotransmitter. Sources: GOC:dph Relationships: is a type of neurotransmitter secretion [GO:0007269]; is_a glutamate secretion [GO:0014047]; is a type of L-glutamate import [GO:0051938]; is part of synaptic transmission, glutamatergic [GO:0035249] Regulation: regulated by regulation of glutamate secretion, neurotransmission [GO:1903294]; negatively regulated by GO:1903295; positively regulated by positive regulation of glutamate secretion, neurotransmission [GO:1903296]